{
  "gene_name": "tRNA (guanine(37)-N1)-methyltransferase",
  "term_label": "mitochondrial matrix",
  "gene_symbol": "TRMT5",
  "gene": "UniProtKB:Q32P41",
  "term_id": "GO:0005759"
}